pyrimidine deoxyribonucleoside diphosphate biosynthetic process [GO:0009197] (BP) Subtypes: dUDP biosynthetic process [GO:0006227], dTDP biosynthetic process [GO:0006233], dCDP biosynthetic process [GO:0006240] Relationships: is a type of pyrimidine nucleoside diphosphate biosynthetic process [GO:0009139]; is_a GO:0009189; is a type of pyrimidine deoxyribonucleoside diphosphate metabolic process [GO:0009196] Also known as: pyrimidine deoxyribonucleoside diphosphate anabolism, pyrimidine deoxyribonucleoside diphosphate biosynthesis, pyrimidine deoxyribonucleoside diphosphate formation, pyrimidine deoxyribonucleoside diphosphate synthesis Definition: The chemical reactions and pathways resulting in the formation of pyrimidine deoxyribonucleoside diphosphate, a compound consisting of a pyrimidine base linked to a deoxyribose sugar esterified with diphosphate on the sugar. Sources: GOC:go_curators, ISBN:0198506732